{
  "term_id": "GO:0005615",
  "gene": "UniProtKB:Q8IZJ0",
  "gene_name": "Interferon lambda-2",
  "gene_symbol": "IFNL2",
  "term_label": "extracellular space"
}